{
  "gene_name": "E3 ubiquitin-protein ligase DZIP3",
  "gene": "UniProtKB:Q86Y13",
  "gene_symbol": "DZIP3",
  "term_label": "protein polyubiquitination",
  "term_id": "GO:0000209"
}